(R)-aminopropanol dehydrogenase activity [GO:0019147] (MF) Also known as: L-aminopropanol dehydrogenase activity, (R)-1-aminopropan-2-ol:NAD+ oxidoreductase activity, 1-aminopropan-2-ol-NAD+ dehydrogenase activity, 1-aminopropan-2-ol-dehydrogenase activity, DL-1-aminopropan-2-ol: NAD+ dehydrogenase activity, L(+)-1-aminopropan-2-ol-NAD/NADP oxidoreductase activity, L(+)-1-aminopropan-2-ol:NAD+ oxidoreductase activity Relationships: is a type of oxidoreductase activity, acting on the CH-OH group of donors, NAD or NADP as acceptor [GO:0016616] Sources: EC:1.1.1.75, RHEA:16517 Definition: Catalysis of the reaction: (R)-1-aminopropan-2-ol + NAD+ = aminoacetone + H+ + NADH.